proline:sodium symporter activity [GO:0005298] (molecular function) Sources: TC:2.A.22.2.1 Also known as: sodium/proline symporter activity Relationships: is a type of GO:0005283; is a type of organic acid:sodium symporter activity [GO:0005343]; is a type of carboxylic acid transmembrane transporter activity [GO:0046943] Definition: Enables the transfer of a solute or solutes from one side of a membrane to the other according to the reaction: proline(out) + Na+(out) = proline(in) + Na+(in).